{
  "term_id": "UNKNOWN:0003",
  "gene": "UniProtKB:Q96C36",
  "term_label": "Unknown cellular component",
  "gene_name": "Pyrroline-5-carboxylate reductase 2",
  "gene_symbol": "PYCR2"
}